{
  "term_label": "establishment or maintenance of apical/basal cell polarity",
  "gene_symbol": "OOEP",
  "term_id": "GO:0035088",
  "gene_name": "Oocyte-expressed protein homolog",
  "gene": "UniProtKB:A6NGQ2"
}